{
  "gene_name": "DNA excision repair protein ERCC-1",
  "term_id": "GO:0000110",
  "gene_symbol": "ERCC1",
  "term_label": "nucleotide-excision repair factor 1 complex",
  "gene": "UniProtKB:P07992"
}